{
  "term_id": "GO:0002178",
  "term_label": "palmitoyltransferase complex",
  "gene_name": "Golgin subfamily A member 7",
  "gene_symbol": "GOLGA7",
  "gene": "UniProtKB:Q7Z5G4"
}